{
  "gene_name": "Histone-lysine N-methyltransferase NSD2",
  "term_id": "GO:0000785",
  "gene": "UniProtKB:O96028",
  "term_label": "chromatin",
  "gene_symbol": "NSD2"
}